negative regulation of pro-B cell differentiation [GO:2000974] (biological process) Definition: Any process that stops, prevents or reduces the frequency, rate or extent of pro-B cell differentiation. Sources: GOC:obol Also known as: negative regulation of pro-B lymphocyte differentiation, negative regulation of pro-B cell development Relationships: is a type of negative regulation of lymphoid progenitor cell differentiation [GO:1905457]; is a type of GO:2000973; negatively regulates pro-B cell differentiation [GO:0002328]